{
  "term_label": "Unknown molecular function",
  "term_id": "UNKNOWN:0001",
  "gene": "UniProtKB:Q5T6V5",
  "gene_symbol": "QNG1",
  "gene_name": "Queuosine 5'-phosphate N-glycosylase_hydrolase"
}